{
  "gene": "UniProtKB:Q9H246",
  "gene_symbol": "C1orf21",
  "term_id": "UNKNOWN:0002",
  "gene_name": "Uncharacterized protein C1orf21",
  "term_label": "Unknown biological process"
}